{
  "term_id": "GO:0000981",
  "gene_symbol": "ZNF160",
  "gene_name": "Zinc finger protein 160",
  "term_label": "DNA-binding transcription factor activity, RNA polymerase II-specific",
  "gene": "UniProtKB:Q9HCG1"
}